{
  "gene_name": "Thymic stromal lymphopoietin",
  "gene_symbol": "TSLP",
  "gene": "UniProtKB:Q969D9",
  "term_label": "positive regulation of inflammatory response",
  "term_id": "GO:0050729"
}